regulation of excitatory synapse pruning [GO:1905810] (biological process) References: PMID:27779093 Sources: GOC:TermGenie, GO_REF:0000058 Also known as: regulation of synapse clearance, regulation of synapse disassembly, regulation of synapse elimination, regulation of synapse removal Subtypes: GO:1905811 Definition: Any process that modulates the frequency, rate or extent of excitatory synapse pruning. Relationships: is a type of regulation of synapse pruning [GO:1905806]; regulates excitatory synapse pruning [GO:1905805]